{
  "term_label": "cytoplasm",
  "gene_symbol": "FGF19",
  "term_id": "GO:0005737",
  "gene_name": "Fibroblast growth factor 19",
  "gene": "UniProtKB:O95750"
}